intracellularly ATP-gated ion channel activity [GO:0099142] (MF) Subtypes: GO:0005260 Relationships: is a type of intracellularly ligand-gated monoatomic ion channel activity [GO:0005217]; is a type of ATP-gated ion channel activity [GO:0035381] References: PMID:9755289 Definition: Enables the transmembrane transfer of an ion by a channel that opens when ATP has been bound by the channel complex or one of its constituent parts on the intracellular side of the plasma membrane.